{
  "term_id": "GO:0005737",
  "gene_name": "Adhesion G-protein coupled receptor V1",
  "term_label": "cytoplasm",
  "gene_symbol": "ADGRV1",
  "gene": "UniProtKB:Q8WXG9"
}